{
  "gene_symbol": "PPP1R14B",
  "gene": "UniProtKB:Q96C90",
  "gene_name": "Protein phosphatase 1 regulatory subunit 14B",
  "term_id": "UNKNOWN:0003",
  "term_label": "Unknown cellular component"
}